{
  "gene_name": "Terminal nucleotidyltransferase 4A",
  "gene_symbol": "TENT4A",
  "gene": "UniProtKB:Q5XG87",
  "term_id": "GO:0031123",
  "term_label": "RNA 3'-end processing"
}